{
  "gene_symbol": "UTP20",
  "term_label": "small-subunit processome",
  "term_id": "GO:0032040",
  "gene_name": "Small subunit processome component 20 homolog",
  "gene": "UniProtKB:O75691"
}